{
  "gene_symbol": "SPACA5",
  "gene_name": "Sperm acrosome-associated protein 5",
  "gene": "UniProtKB:Q96QH8",
  "term_label": "acrosomal vesicle",
  "term_id": "GO:0001669"
}